{
  "gene": "UniProtKB:Q99788",
  "gene_symbol": "CMKLR1",
  "term_label": "complement receptor activity",
  "term_id": "GO:0004875",
  "gene_name": "Chemerin-like receptor 1"
}